{
  "term_id": "GO:0050839",
  "term_label": "cell adhesion molecule binding",
  "gene_symbol": "CXADR",
  "gene_name": "Coxsackievirus and adenovirus receptor",
  "gene": "UniProtKB:P78310"
}